xanthophore differentiation [GO:0050936] (biological process) Relationships: is a type of pigment cell differentiation [GO:0050931] References: PMID:11858836 Sources: GOC:jid, GOC:mh Note: Note that this term refers to xanthophores in the sense of specialized pigment-producing cells, and should not be confused with the cellular component term 'xanthophore ; GO:0031633', which refers to a subcellular structure. Definition: The process in which a relatively unspecialized cell acquires the specialized features of a xanthophore cell. Xanthophores are pigment cells derived from the neural crest. They contain pteridine and/or carotenoid pigments in structures called pterinosomes or xanthosomes. This makes them yellow to orange in appearance. Regulation: regulated by GO:0050938; negatively regulated by negative regulation of xanthophore differentiation [GO:0050944]; RO_0002213 by positive regulation of xanthophore differentiation [GO:0050946] Also known as: xanthophore cell differentiation